{
  "gene": "UniProtKB:P38435",
  "gene_symbol": "GGCX",
  "term_id": "GO:0019842",
  "gene_name": "Vitamin K-dependent gamma-carboxylase",
  "term_label": "vitamin binding"
}